{
  "term_id": "GO:0006511",
  "term_label": "ubiquitin-dependent protein catabolic process",
  "gene_name": "Cullin-9",
  "gene": "UniProtKB:Q8IWT3",
  "gene_symbol": "CUL9"
}